{
  "gene_name": "Ecto-ADP-ribosyltransferase 4",
  "term_label": "Unknown biological process",
  "gene_symbol": "ART4",
  "gene": "UniProtKB:Q93070",
  "term_id": "UNKNOWN:0002"
}